{
  "gene": "UniProtKB:Q15726",
  "gene_name": "Metastasis-suppressor KiSS-1",
  "term_id": "GO:0031773",
  "gene_symbol": "KISS1",
  "term_label": "kisspeptin receptor binding"
}